{
  "gene_symbol": "IFIT1",
  "term_id": "GO:0071345",
  "gene": "UniProtKB:P09914",
  "term_label": "cellular response to cytokine stimulus",
  "gene_name": "Interferon-induced protein with tetratricopeptide repeats 1"
}